{
  "term_label": "spindle organization",
  "term_id": "GO:0007051",
  "gene_symbol": "NTMT1",
  "gene": "UniProtKB:Q9BV86",
  "gene_name": "N-terminal Xaa-Pro-Lys N-methyltransferase 1"
}